flower phyllotactic patterning [GO:0060773] (biological process) Definition: The radial pattern formation process that results in the formation of floral organ primordia around a central axis in a flower primordium. Sources: GOC:dph, GOC:sdb_2009, GOC:tb Relationships: is a type of phyllotactic patterning [GO:0060771]